{
  "gene_name": "Mitogen-activated protein kinase 8",
  "gene_symbol": "MAPK8",
  "gene": "UniProtKB:P45983",
  "term_id": "GO:0005737",
  "term_label": "cytoplasm"
}